2-methyleneglutarate mutase activity [GO:0047548] (molecular function) Also known as: 2-methyleneglutarate carboxy-methylenemethylmutase activity, alpha-methyleneglutarate mutase activity Relationships: is a type of intramolecular transferase activity [GO:0016866] Sources: EC:5.4.99.4, RHEA:13793 Definition: Catalysis of the reaction: 2-methyleneglutarate = 2-methylene-3-methylsuccinate.